progression of neural tube closure [GO:0021994] (biological process) Definition: The process in which the neural folds are fused extending from the initial closure points. Relationships: is a type of morphogenesis of embryonic epithelium [GO:0016331]; is part of neural tube closure [GO:0001843] Sources: GOC:cls, GOC:dgh, GOC:dph, GOC:jid, GO_REF:0000021